{
  "term_label": "Unknown biological process",
  "gene_symbol": "NBPF7P",
  "gene": "UniProtKB:P0C2Y1",
  "gene_name": "Putative neuroblastoma breakpoint family member 7",
  "term_id": "UNKNOWN:0002"
}